{
  "term_label": "ceramide biosynthetic process",
  "gene_symbol": "DEGS2",
  "gene": "UniProtKB:Q6QHC5",
  "gene_name": "Sphingolipid delta(4)-desaturase_C4-monooxygenase DES2",
  "term_id": "GO:0046513"
}